anti-Mullerian hormone receptor signaling pathway [GO:1990262] (BP) References: PMID:23624077 Sources: GOC:hjd Definition: The series of molecular signals initiated by the binding of anti-Mullerian hormone to its receptor on the surface of a target cell, and ending with the regulation of a downstream cellular process, e.g. transcription. Upon ligand binding, the receptor  forms a complex consisting of two type II and two type I transmembrane serine/threonine kinases. Type II receptors phosphorylate and activate type I receptors which autophosphorylate, then bind and activate SMAD transcriptional regulators. Relationships: is a type of GO:0007178 Regulation: regulated by GO:1902612; negatively regulated by negative regulation of anti-Mullerian hormone signaling pathway [GO:1902613]; positively regulated by positive regulation of anti-Mullerian hormone signaling pathway [GO:1902614] Also known as: anti-Mullerian hormone signaling pathway Note: An example of this is Amhr2 in M. musculus (Q8K592) a receptor for anti-mullerian hormone, described in PMID:23624077.